{
  "gene": "UniProtKB:Q9H867",
  "term_label": "protein-lysine N-methyltransferase activity",
  "gene_symbol": "VCPKMT",
  "gene_name": "Protein N-lysine methyltransferase METTL21D",
  "term_id": "GO:0016279"
}